{
  "gene_symbol": "IFNL4",
  "gene": "UniProtKB:K9M1U5",
  "gene_name": "Interferon lambda-4",
  "term_label": "signaling receptor binding",
  "term_id": "GO:0005102"
}